{
  "gene": "UniProtKB:Q4VXU2",
  "gene_name": "Polyadenylate-binding protein 1-like",
  "term_label": "cytosol",
  "gene_symbol": "PABPC1L",
  "term_id": "GO:0005829"
}